{
  "term_label": "protein kinase binding",
  "term_id": "GO:0019901",
  "gene_name": "Rho-related GTP-binding protein Rho6",
  "gene_symbol": "RND1",
  "gene": "UniProtKB:Q92730"
}